{
  "gene_symbol": "BAIAP2",
  "term_label": "cytosol",
  "gene": "UniProtKB:Q9UQB8",
  "term_id": "GO:0005829",
  "gene_name": "Brain-specific angiogenesis inhibitor 1-associated protein 2"
}